{
  "gene_symbol": "ABHD3",
  "term_id": "GO:0051792",
  "term_label": "medium-chain fatty acid biosynthetic process",
  "gene_name": "Phospholipase ABHD3",
  "gene": "UniProtKB:Q8WU67"
}